{
  "term_label": "RNA polymerase II complex binding",
  "gene": "UniProtKB:Q96P16",
  "gene_symbol": "RPRD1A",
  "gene_name": "Regulation of nuclear pre-mRNA domain-containing protein 1A",
  "term_id": "GO:0000993"
}